{
  "gene_name": "Nicastrin",
  "term_id": "GO:0005886",
  "gene": "UniProtKB:Q92542",
  "term_label": "plasma membrane",
  "gene_symbol": "NCSTN"
}